{
  "gene_symbol": "ZFAND1",
  "term_label": "stress granule disassembly",
  "gene_name": "AN1-type zinc finger protein 1",
  "gene": "UniProtKB:Q8TCF1",
  "term_id": "GO:0035617"
}